Purkinje myocyte to ventricular cardiac muscle cell signaling [GO:0086029] (biological process) Definition: Any process that mediates the transfer of information from a Purkinje myocyte to a ventricular cardiac muscle cell. Sources: GOC:BHF, GOC:mtg_cardiac_conduct_nov11 Relationships: is a type of cell-cell signaling involved in cardiac conduction [GO:0086019]; is a type of Purkinje myocyte to ventricular cardiac muscle cell communication [GO:0086068] Also known as: Purkinje myocyte to ventricular cardiac muscle cell signalling